propionate metabolic process [GO:0019541] (biological process) Also known as: propanoate metabolic process, propanoate metabolism, propionate metabolism Subtypes: GO:0019542, GO:0019543, lactate fermentation to propionate and acetate [GO:0019652], pyruvate fermentation to propionate [GO:0019657], GO:0019678, propionate metabolic process, methylcitrate cycle [GO:0019679], L-glutamate catabolic process to propionate [GO:0033509], GO:0070689 Sources: GOC:go_curators, ISBN:0198506732 Definition: The chemical reactions and pathways involving propionate, the anion derived from propionic (propanoic) acid, a carboxylic acid important in the energy metabolism of ruminants. Relationships: is a type of short-chain fatty acid metabolic process [GO:0046459]